{
  "gene_symbol": "MMP23B",
  "gene": "UniProtKB:O75900",
  "term_id": "GO:0030574",
  "term_label": "collagen catabolic process",
  "gene_name": "Matrix metalloproteinase-23"
}